{
  "gene": "UniProtKB:Q8NEM7",
  "term_label": "SAGA complex",
  "gene_symbol": "SUPT20H",
  "gene_name": "Transcription factor SPT20 homolog",
  "term_id": "GO:0000124"
}